{
  "gene": "UniProtKB:P35869",
  "term_label": "nuclear receptor activity",
  "gene_name": "Aryl hydrocarbon receptor",
  "gene_symbol": "AHR",
  "term_id": "GO:0004879"
}